primary metabolic process [GO:0044238] (biological process) Sources: GOC:go_curators Also known as: primary metabolism Definition: The chemical reactions and pathways involving those compounds which are formed as a part of the normal anabolic and catabolic processes. These processes take place in most, if not all, cells of the organism. Subtypes: GO:0005975, tricarboxylic acid cycle [GO:0006099], nucleobase-containing compound metabolic process [GO:0006139], RNA processing [GO:0006396], amino acid metabolic process [GO:0006520], lipid metabolic process [GO:0006629], GO:0019538, phytochelatin metabolic process [GO:0046937] Relationships: is a type of GO:0008152 Regulation: regulated by GO:0080090